polyphosphate metabolic process [GO:0006797] (BP) Subtypes: polyphosphate catabolic process [GO:0006798], polyphosphate biosynthetic process [GO:0006799] Sources: GOC:go_curators, ISBN:0198506732 Definition: The chemical reactions and pathways involving a polyphosphate, the anion or salt of polyphosphoric acid. Relationships: is a type of phosphorus metabolic process [GO:0006793]; is a type of oxoacid metabolic process [GO:0043436] Also known as: polyphosphate metabolism